selenomethionine gamma-lyase activity [GO:0098600] (molecular function) Definition: Catalysis of the reaction: L-Selenomethionine + H2O = Methaneselenol + Ammonia + 2-oxobutanoic acid. References: PMID:11578145, PMID:16037612, PMID:16444005 Relationships: is_a GO:0016846